{
  "term_id": "GO:0006357",
  "gene_symbol": "YEATS2",
  "gene_name": "YEATS domain-containing protein 2",
  "gene": "UniProtKB:Q9ULM3",
  "term_label": "regulation of transcription by RNA polymerase II"
}